{
  "term_id": "GO:0005525",
  "gene": "UniProtKB:P51159",
  "gene_symbol": "RAB27A",
  "term_label": "GTP binding",
  "gene_name": "Ras-related protein Rab-27A"
}